{
  "gene": "UniProtKB:A0A0A0MT69",
  "gene_symbol": "IGKJ4",
  "term_id": "UNKNOWN:0001",
  "term_label": "Unknown molecular function",
  "gene_name": "Immunoglobulin kappa joining 4 (Fragment)"
}